epi-isozizaene synthase activity [GO:0052680] (molecular function) Also known as: (2E,6E)-farnesyl-diphosphate diphosphate-lyase [(+)-epi-isozizaene-forming] activity Sources: RHEA:25992 Definition: Catalysis of the reaction: 2-trans,6-trans-farnesyl diphosphate = (+)-epi-isozizaene + diphosphate. Relationships: is a type of GO:0016838